{
  "term_label": "RNA polymerase II general transcription initiation factor activity",
  "gene": "UniProtKB:P35269",
  "gene_symbol": "GTF2F1",
  "gene_name": "General transcription factor IIF subunit 1",
  "term_id": "GO:0016251"
}